{
  "gene_symbol": "PLA2G4A",
  "gene_name": "Cytosolic phospholipase A2",
  "term_label": "nucleus",
  "gene": "UniProtKB:P47712",
  "term_id": "GO:0005634"
}